{
  "gene_name": "Leucine-rich repeat-containing protein 30",
  "gene_symbol": "LRRC30",
  "gene": "UniProtKB:A6NM36",
  "term_label": "Unknown cellular component",
  "term_id": "UNKNOWN:0003"
}